{
  "gene_symbol": "KLRG1",
  "term_id": "UNKNOWN:0003",
  "term_label": "Unknown cellular component",
  "gene": "UniProtKB:Q96E93",
  "gene_name": "Killer cell lectin-like receptor subfamily G member 1"
}